{
  "gene_name": "Protein ZGRF1",
  "term_id": "UNKNOWN:0001",
  "gene_symbol": "ZGRF1",
  "gene": "UniProtKB:Q86YA3",
  "term_label": "Unknown molecular function"
}